{
  "term_label": "Unknown biological process",
  "gene": "UniProtKB:Q8N5S3",
  "term_id": "UNKNOWN:0002",
  "gene_name": "Uncharacterized protein C2orf73",
  "gene_symbol": "C2orf73"
}